regulation of antigen processing and presentation of endogenous peptide antigen via MHC class I [GO:1904282] (biological process) Also known as: regulation of antigen presentation, endogenous peptide antigen, regulation of antigen processing, endogenous antigen via MHC class I, regulation of antigen processing, endogenous antigen via major histocompatibility complex class I, regulation of endogenous peptide antigen processing and presentation via MHC class I References: PMID:24643698 Sources: GOC:BHF, GOC:TermGenie, GOC:rl, GO_REF:0000058 Subtypes: negative regulation of antigen processing and presentation of endogenous peptide antigen via MHC class I [GO:1904283], positive regulation of antigen processing and presentation of endogenous peptide antigen via MHC class I [GO:1904284] Relationships: is a type of GO:0002589; regulates antigen processing and presentation of endogenous peptide antigen via MHC class I [GO:0019885] Definition: Any process that modulates the frequency, rate or extent of antigen processing and presentation of endogenous peptide antigen via MHC class I.